hydroxypyruvate reductase [NAD(P)H] activity [GO:0016618] (molecular function) Subtypes: hydroxypyruvate reductase (NADH) activity [GO:0008465], hydroxypyruvate reductase (NADPH) activity [GO:0120509] Sources: EC:1.1.1.81 Also known as: hydroxypyruvate reductase activity, D-glycerate dehydrogenase activity, D-glycerate:NADP+ 2-oxidoreductase activity, NADH:hydroxypyruvate reductase activity, beta-hydroxypyruvate reductase activity Relationships: is a type of oxidoreductase activity, acting on the CH-OH group of donors, NAD or NADP as acceptor [GO:0016616] Definition: Catalysis of the reaction: (R)-glycerate + NAD(P)+ = 3-hydroxypyruvate + NAD(P)H + H+.